{
  "term_label": "Unknown biological process",
  "term_id": "UNKNOWN:0002",
  "gene_name": "Protein-L-histidine N-pros-methyltransferase",
  "gene": "UniProtKB:Q9H1A3",
  "gene_symbol": "METTL9"
}